regulation of very-low-density lipoprotein particle clearance [GO:0010915] (biological process) Definition: Any process that modulates the rate, frequency or extent of very-low-density lipoprotein particle clearance. Very-low-density lipoprotein particle clearance is the process in which a very-low-density lipoprotein particle is removed from the blood via receptor-mediated endocytosis and its constituent parts degraded. Subtypes: negative regulation of very-low-density lipoprotein particle clearance [GO:0010916], positive regulation of very-low-density lipoprotein particle clearance [GO:0110119] Relationships: is a type of regulation of lipoprotein particle clearance [GO:0010984]; regulates very-low-density lipoprotein particle clearance [GO:0034447] Sources: GOC:BHF, GOC:dph, GOC:tb Also known as: regulation of VLDL clearance, regulation of VLDL particle clearance